{
  "term_id": "GO:0019005",
  "gene_name": "F-box_LRR-repeat protein 2",
  "term_label": "SCF ubiquitin ligase complex",
  "gene_symbol": "FBXL2",
  "gene": "UniProtKB:Q9UKC9"
}